{
  "term_label": "calcium ion binding",
  "gene": "UniProtKB:Q9Y2W7",
  "term_id": "GO:0005509",
  "gene_name": "Calsenilin",
  "gene_symbol": "KCNIP3"
}